{
  "gene_symbol": "TRAV29DV5",
  "term_id": "UNKNOWN:0003",
  "gene": "UniProtKB:P04437",
  "term_label": "Unknown cellular component",
  "gene_name": "T cell receptor alpha variable 29_delta variable 5"
}